{
  "gene_symbol": "TUBD1",
  "gene_name": "Tubulin delta chain",
  "term_label": "cytoplasm",
  "term_id": "GO:0005737",
  "gene": "UniProtKB:Q9UJT1"
}